{
  "term_label": "iron-sulfur cluster assembly",
  "gene": "UniProtKB:Q9Y5Y2",
  "gene_name": "Cytosolic Fe-S cluster assembly factor NUBP2",
  "gene_symbol": "NUBP2",
  "term_id": "GO:0016226"
}